{
  "gene": "UniProtKB:Q9NUU7",
  "term_label": "mRNA binding",
  "term_id": "GO:0003729",
  "gene_name": "ATP-dependent RNA helicase DDX19A",
  "gene_symbol": "DDX19A"
}